chloroplast fission [GO:0010020] (biological process) Also known as: chloroplast division Sources: GOC:lr Relationships: is a type of chloroplast organization [GO:0009658]; is a type of plastid fission [GO:0043572] Regulation: regulated by GO:1905192; negatively regulated by negative regulation of chloroplast fission [GO:1905193]; positively regulated by positive regulation of chloroplast fission [GO:1905194] Definition: The division of a chloroplast within a cell to form two or more separate chloroplast compartments. This division occurs independently of mitosis.